host cell surface binding [GO:0046812] (molecular function) Definition: Binding to the surface of a host cell. Sources: GOC:ai Subtypes: GO:0046789 Relationships: is a type of binding [GO:0005488]